positive regulation of central B cell deletion [GO:0002900] (biological process) Definition: Any process that activates or increases the frequency, rate, or extent of central B cell deletion. Relationships: is a type of positive regulation of B cell deletion [GO:0002869]; is_a positive regulation of central B cell tolerance induction [GO:0002897]; is a type of regulation of central B cell deletion [GO:0002898]; is a type of positive regulation of B cell differentiation [GO:0045579]; RO_0002213 central B cell deletion [GO:0002342] Also known as: up regulation of central B cell deletion, up-regulation of central B cell deletion, upregulation of central B cell deletion, activation of central B cell deletion, stimulation of central B cell deletion Sources: GOC:add